{
  "term_label": "calcium ion binding",
  "gene_name": "Desmocollin-3",
  "gene_symbol": "DSC3",
  "term_id": "GO:0005509",
  "gene": "UniProtKB:Q14574"
}